{
  "gene": "UniProtKB:P21730",
  "gene_symbol": "C5AR1",
  "term_label": "inflammatory response",
  "gene_name": "C5a anaphylatoxin chemotactic receptor 1",
  "term_id": "GO:0006954"
}